urate:monoatomic anion antiporter activity [GO:0140813] (molecular function) Definition: Enables the transfer of a solute or solutes from one side of a membrane to the other according to the reaction: urate(out) + anion (in) = urate (in) + anion (out). Relationships: is a type of monoatomic anion transmembrane transporter activity [GO:0008509]; is a type of antiporter activity [GO:0015297]; is part of urate transport [GO:0015747] References: PMID:12024214, PMID:18411268 Also known as: urate:anion antiporter activity, urate:organic anion antiporter activity